regulation of meristem growth [GO:0010075] (biological process) Relationships: is a type of regulation of developmental growth [GO:0048638]; is part of meristem maintenance [GO:0010073]; regulates GO:0035266 Sources: GOC:tb Subtypes: homeostasis of number of meristem cells [GO:0007639], regulation of floral meristem growth [GO:0010080], GO:0010081, GO:0010082, regulation of vegetative meristem growth [GO:0010083] Definition: Any process involved in maintaining the size and shape of a meristem. Also known as: regulation of meristem size